aminoglycan metabolic process [GO:0006022] (BP) Subtypes: aminoglycan biosynthetic process [GO:0006023], aminoglycan catabolic process [GO:0006026], chitin metabolic process [GO:0006030], glycosaminoglycan metabolic process [GO:0030203], poly-N-acetyllactosamine metabolic process [GO:0030309] Definition: The chemical reactions and pathways involving aminoglycans, any polymer containing amino groups that consists of more than about 10 monosaccharide residues joined to each other by glycosidic linkages. Also known as: aminoglycan metabolism Sources: GOC:ai, ISBN:0198506732 Relationships: is a type of GO:0043170; is a type of carbohydrate derivative metabolic process [GO:1901135]